protein import into mitochondrial matrix [GO:0030150] (BP) Relationships: is a type of protein localization to mitochondrion [GO:0070585]; is a type of protein transmembrane transport [GO:0071806]; is a type of establishment of protein localization to mitochondrion [GO:0072655] Sources: ISBN:0716731363 Definition: The import of proteins across the outer and inner mitochondrial membranes into the matrix. Unfolded proteins enter the mitochondrial matrix with a chaperone protein; the information required to target the precursor protein from the cytosol to the mitochondrial matrix is contained within its N-terminal matrix-targeting sequence. Translocation of precursors to the matrix occurs at the rare sites where the outer and inner membranes are close together. Also known as: mitochondrial translocation, mitochondrial matrix protein import, protein transport into mitochondrial matrix